sigma factor antagonist complex [GO:1903865] (cellular component) Definition: A protein complex which is capable of sigma factor antagonist activity. Relationships: is a type of transcription regulator complex [GO:0005667] References: PMID:23687042 Sources: GOC:TermGenie, GOC:bhm, GO_REF:0000088